{
  "gene": "UniProtKB:Q6PKC3",
  "term_id": "UNKNOWN:0003",
  "gene_name": "Thioredoxin domain-containing protein 11",
  "term_label": "Unknown cellular component",
  "gene_symbol": "TXNDC11"
}